{
  "term_id": "GO:0019731",
  "gene_symbol": "IGHE",
  "gene_name": "Immunoglobulin heavy constant epsilon",
  "term_label": "antibacterial humoral response",
  "gene": "UniProtKB:P01854"
}